{
  "gene_name": "Gamma-taxilin",
  "gene_symbol": "TXLNG",
  "term_id": "UNKNOWN:0001",
  "gene": "UniProtKB:Q9NUQ3",
  "term_label": "Unknown molecular function"
}